smooth muscle atrophy [GO:0014890] (biological process) Definition: A process, occurring in smooth muscle, that is characterized by a decrease in protein content, fiber diameter, force production and fatigue resistance in response to different conditions such as starvation, aging and disuse. Sources: GOC:mtg_muscle Relationships: is a type of smooth muscle adaptation [GO:0014805]; is a type of muscle atrophy [GO:0014889]